{
  "term_label": "peptide antigen binding",
  "gene_symbol": "HLA-DOB",
  "term_id": "GO:0042605",
  "gene": "UniProtKB:P13765",
  "gene_name": "HLA class II histocompatibility antigen, DO beta chain"
}